{
  "gene_symbol": "IGHV3-38",
  "gene": "UniProtKB:A0A0C4DH36",
  "gene_name": "Probable non-functional immunoglobulin heavy variable 3-38",
  "term_id": "GO:0016064",
  "term_label": "immunoglobulin mediated immune response"
}